negative regulation of telomere maintenance via telomerase [GO:0032211] (biological process) Definition: Any process that stops, prevents, or reduces the frequency, rate or extent of the addition of telomeric repeats by telomerase. Relationships: is a type of regulation of telomere maintenance via telomerase [GO:0032210]; is a type of negative regulation of telomere maintenance via telomere lengthening [GO:1904357]; is a type of negative regulation of DNA biosynthetic process [GO:2000279]; negatively regulates telomere maintenance via telomerase [GO:0007004] Sources: GOC:mah Also known as: down regulation of telomere maintenance via telomerase activity, down-regulation of telomere maintenance via telomerase activity, downregulation of telomere maintenance via telomerase activity, inhibition of telomere maintenance via telomerase